{
  "gene": "UniProtKB:Q8NDX5",
  "gene_symbol": "PHC3",
  "term_id": "GO:0045892",
  "gene_name": "Polyhomeotic-like protein 3",
  "term_label": "negative regulation of DNA-templated transcription"
}